{
  "term_id": "UNKNOWN:0002",
  "gene": "UniProtKB:Q537H7",
  "term_label": "Unknown biological process",
  "gene_symbol": "SPATA45",
  "gene_name": "Spermatogenesis-associated protein 45"
}